{
  "term_label": "A band",
  "term_id": "GO:0031672",
  "gene_name": "Myosin light chain 4",
  "gene_symbol": "MYL4",
  "gene": "UniProtKB:P12829"
}